axon regeneration at neuromuscular junction [GO:0014814] (biological process) Sources: GOC:ef, GOC:mtg_muscle Relationships: is a type of axon regeneration [GO:0031103] Definition: The regrowth of axons following their loss or damage at the neuromuscular junction. Motor axons regenerate after injury and they form neuro-muscular junctions with skeletal myofibers similar to normal ones.